{
  "gene_name": "Cytoplasmic polyadenylated homeobox-like protein 2",
  "term_id": "GO:0000981",
  "gene_symbol": "CPHXL2",
  "gene": "UniProtKB:A0A1W2PPK0",
  "term_label": "DNA-binding transcription factor activity, RNA polymerase II-specific"
}